{
  "gene_symbol": "BSN",
  "gene_name": "Protein bassoon",
  "term_id": "GO:0098982",
  "term_label": "GABA-ergic synapse",
  "gene": "UniProtKB:Q9UPA5"
}